regulation of mating type switching [GO:0031494] (biological process) Definition: Any process that modulates the frequency, rate or extent of mating type switching, the conversion of a single-cell organism from one mating type to another by the precise replacement of a DNA sequence at the expressed mating type locus with a copy of a sequence from a donor locus. Sources: GOC:mah Relationships: is a type of regulation of developmental process [GO:0050793]; is a type of GO:2000241; regulates GO:0007533 Subtypes: GO:0031495, positive regulation of mating type switching [GO:0031496]